negative regulation of protein catabolic process [GO:0042177] (biological process) Also known as: down regulation of cellular protein breakdown, down regulation of cellular protein catabolic process, down regulation of cellular protein catabolism, down regulation of cellular protein degradation, down regulation of protein catabolic process, down-regulation of cellular protein breakdown, down-regulation of cellular protein catabolic process, down-regulation of cellular protein catabolism, down-regulation of cellular protein degradation, down-regulation of protein catabolic process, downregulation of cellular protein breakdown, downregulation of cellular protein catabolic process, downregulation of cellular protein catabolism, downregulation of cellular protein degradation, downregulation of protein catabolic process, negative regulation of cellular protein breakdown, negative regulation of cellular protein catabolic process, negative regulation of cellular protein catabolism, negative regulation of cellular protein degradation, negative regulation of protein breakdown, negative regulation of protein catabolism, negative regulation of protein degradation, inhibition of cellular protein breakdown, inhibition of cellular protein catabolic process, inhibition of cellular protein catabolism, inhibition of cellular protein degradation, inhibition of protein catabolic process Subtypes: negative regulation of proteolysis associated with antigen processing and presentation [GO:0002629], negative regulation of low-density lipoprotein particle receptor catabolic process [GO:0032804], negative regulation of membrane protein ectodomain proteolysis [GO:0051045], negative regulation of elastin catabolic process [GO:0060311], negative regulation of proteasomal protein catabolic process [GO:1901799], negative regulation of protein catabolic process in the vacuole [GO:1904351], negative regulation of chaperone-mediated autophagy [GO:1904715] References: PMID:24785082 Sources: GOC:TermGenie, GOC:kmv, GOC:obol, GO_REF:0000058 Definition: Any process that stops, prevents or reduces the frequency, rate or extent of protein catabolic process. Relationships: is a type of GO:0009895; is a type of regulation of protein catabolic process [GO:0042176]; is_a negative regulation of protein metabolic process [GO:0051248]; negatively regulates GO:0030163